modulation by symbiont of entry into host [GO:0052372] (biological process) Also known as: modulation by organism of entry into other organism during symbiotic interaction, regulation by organism of entry into other organism during symbiotic interaction, regulation by organism of entry into other organism involved in symbiotic interaction Subtypes: regulation of viral entry into host cell [GO:0046596], modulation of penetration peg formation [GO:0075054], modulation of symbiont haustorium neck formation for entry into host [GO:0075198], regulation of penetration hypha formation [GO:0075202], positive regulation by symbiont of entry into host [GO:0075294], regulation of entry of bacterium into host cell [GO:2000535] Definition: Any process in which an organism modulates the frequency, rate or extent to which it enters into the host organism, where the two organisms are in a symbiotic interaction. Relationships: is a type of regulation of biological process involved in symbiotic interaction [GO:0043903]; regulates GO:0044409 Sources: GOC:mtg_pamgo_17jul06